{
  "term_id": "GO:0050830",
  "term_label": "defense response to Gram-positive bacterium",
  "gene_name": "Ribonuclease 4",
  "gene_symbol": "RNASE4",
  "gene": "UniProtKB:P34096"
}